{
  "gene_symbol": "LRRC19",
  "term_id": "GO:0002224",
  "term_label": "toll-like receptor signaling pathway",
  "gene": "UniProtKB:Q9H756",
  "gene_name": "Leucine-rich repeat-containing protein 19"
}